{
  "gene": "UniProtKB:Q92934",
  "gene_name": "Bcl2-associated agonist of cell death",
  "gene_symbol": "BAD",
  "term_label": "positive regulation of apoptotic process",
  "term_id": "GO:0043065"
}